lymph gland plasmatocyte differentiation [GO:0035169] (biological process) Also known as: lymph gland plasmatocyte cell differentiation Definition: The process in which a relatively unspecialized larval lymph gland-derived hemocyte precursor cell acquires the specialized features of the phagocytic blood-cell type, the plasmatocyte. Relationships: is a type of GO:0035168; is a type of plasmatocyte differentiation [GO:0042387] References: PMID:11921077, PMID:8174791 Sources: GOC:bf